{
  "term_label": "Unknown cellular component",
  "term_id": "UNKNOWN:0003",
  "gene_symbol": "GNA15",
  "gene_name": "Guanine nucleotide-binding protein subunit alpha-15",
  "gene": "UniProtKB:P30679"
}